R2/R5 cell fate commitment [GO:0007463] (biological process) Definition: The process in which the R2/R5 photoreceptors commit to their cell fate. R2 and R5 are paired photoreceptors which contribute the outer rhabdomeres. References: PMID:3076112, PMID:3937883 Relationships: is a type of compound eye photoreceptor fate commitment [GO:0001752]; is part of R2/R5 cell differentiation [GO:0048054]